{
  "term_id": "UNKNOWN:0001",
  "gene_name": "Multimerin-1",
  "gene_symbol": "MMRN1",
  "gene": "UniProtKB:Q13201",
  "term_label": "Unknown molecular function"
}